{
  "gene_name": "Pleckstrin homology domain-containing family A member 8",
  "term_id": "GO:0035621",
  "gene": "UniProtKB:Q96JA3",
  "term_label": "ER to Golgi ceramide transport",
  "gene_symbol": "PLEKHA8"
}